{
  "term_id": "GO:0016485",
  "gene_name": "Enteropeptidase",
  "gene_symbol": "TMPRSS15",
  "gene": "UniProtKB:P98073",
  "term_label": "protein processing"
}